{
  "term_id": "GO:0046314",
  "gene": "UniProtKB:P17540",
  "gene_name": "Creatine kinase S-type, mitochondrial",
  "gene_symbol": "CKMT2",
  "term_label": "phosphocreatine biosynthetic process"
}